{
  "gene": "UniProtKB:Q14749",
  "gene_name": "Glycine N-methyltransferase",
  "term_label": "S-adenosylmethionine metabolic process",
  "term_id": "GO:0046500",
  "gene_symbol": "GNMT"
}